{
  "term_id": "GO:0015271",
  "term_label": "outward rectifier potassium channel activity",
  "gene": "UniProtKB:Q9NYG8",
  "gene_symbol": "KCNK4",
  "gene_name": "Potassium channel subfamily K member 4"
}